{
  "gene_symbol": "EVX1",
  "gene": "UniProtKB:P49640",
  "gene_name": "Homeobox even-skipped homolog protein 1",
  "term_label": "DNA-binding transcription factor activity, RNA polymerase II-specific",
  "term_id": "GO:0000981"
}